{
  "term_label": "cytoplasm",
  "gene": "UniProtKB:Q13287",
  "gene_symbol": "NMI",
  "gene_name": "N-myc-interactor",
  "term_id": "GO:0005737"
}